Ras guanyl-nucleotide exchange factor complex [GO:1905742] (cellular component) Definition: A protein complex which is capable of Ras guanyl-nucleotide exchange factor activity. References: PMID:20493808 Sources: GOC:TermGenie, GOC:rjd, GO_REF:0000088 Relationships: is a type of GO:0032991